{
  "gene": "UniProtKB:Q7L9B9",
  "gene_name": "Endonuclease_exonuclease_phosphatase family domain-containing protein 1",
  "gene_symbol": "EEPD1",
  "term_id": "UNKNOWN:0001",
  "term_label": "Unknown molecular function"
}